{
  "gene": "UniProtKB:Q9H9D4",
  "gene_symbol": "ZNF408",
  "gene_name": "Zinc finger protein 408",
  "term_label": "DNA-binding transcription factor activity, RNA polymerase II-specific",
  "term_id": "GO:0000981"
}